{
  "gene": "UniProtKB:Q86T65",
  "term_id": "GO:0048715",
  "gene_name": "Disheveled-associated activator of morphogenesis 2",
  "term_label": "negative regulation of oligodendrocyte differentiation",
  "gene_symbol": "DAAM2"
}